{
  "gene_name": "Epithelial-stromal interaction protein 1",
  "gene": "UniProtKB:Q96J88",
  "term_id": "UNKNOWN:0002",
  "term_label": "Unknown biological process",
  "gene_symbol": "EPSTI1"
}